{
  "gene": "UniProtKB:Q3ZCX4",
  "term_id": "GO:0000978",
  "term_label": "RNA polymerase II cis-regulatory region sequence-specific DNA binding",
  "gene_symbol": "ZNF568",
  "gene_name": "Zinc finger protein 568"
}